myosin IV complex [GO:0031474] (CC) Definition: A myosin complex containing one or more class IV myosin heavy chains and associated light chains; myosin IV is relatively uncharacterized, but is predicted to have a single motor domain, one IQ motif and a tail with a Myosin Tail Homology (myTH4) domain homologous to that in the tails of myosins VII and XV. Sources: Wikipedia:Myosin Relationships: is a type of GO:0016461